{
  "term_id": "GO:0042632",
  "term_label": "cholesterol homeostasis",
  "gene": "UniProtKB:P11597",
  "gene_symbol": "CETP",
  "gene_name": "Cholesteryl ester transfer protein"
}